{
  "gene_name": "Rhox homeobox family member 2B",
  "gene_symbol": "RHOXF2B",
  "term_id": "GO:0000981",
  "gene": "UniProtKB:P0C7M4",
  "term_label": "DNA-binding transcription factor activity, RNA polymerase II-specific"
}